neoxanthin biosynthetic process [GO:1901833] (biological process) Relationships: is a type of GO:0016123; is a type of epoxide metabolic process [GO:0097176]; is a type of olefinic compound biosynthetic process [GO:0120255]; is a type of GO:1901503 References: PMID:11029576 Sources: GOC:TermGenie, GOC:yaf, MetaCyc:PWY-6809, UniPathway:UPA00388 Definition: The chemical reactions and pathways resulting in the formation of trans-neoxanthin and 9'-cis-neoxanthin. Also known as: all-trans-neoxanthin anabolism, all-trans-neoxanthin biosynthesis, all-trans-neoxanthin formation, all-trans-neoxanthin synthesis, neoxanthin anabolism, neoxanthin biosynthesis, neoxanthin formation, neoxanthin synthesis, all-trans-neoxanthin biosynthetic process